{
  "gene_symbol": "OR2A25",
  "term_label": "odorant binding",
  "gene_name": "Olfactory receptor 2A25",
  "gene": "UniProtKB:A4D2G3",
  "term_id": "GO:0005549"
}